negative regulation of cell proliferation involved in mesonephros development [GO:2000607] (biological process) Subtypes: GO:2000091 Definition: Any process that stops, prevents or reduces the frequency, rate or extent of cell proliferation involved in mesonephros development. Relationships: is a type of GO:1901723; is a type of regulation of cell proliferation involved in mesonephros development [GO:2000606]; negatively regulates cell proliferation involved in mesonephros development [GO:0061209] Sources: GOC:obol